regulation of toluene catabolic process [GO:1901434] (biological process) Sources: GOC:TermGenie, GOC:mengo_curators Relationships: is a type of regulation of catabolic process [GO:0009894]; regulates GO:0042203 Definition: Any process that modulates the frequency, rate or extent of toluene catabolic process. Subtypes: GO:1901435, positive regulation of toluene catabolic process [GO:1901436] Also known as: regulation of toluene breakdown, regulation of toluene catabolism, regulation of toluene degradation